{
  "gene": "UniProtKB:Q99501",
  "term_id": "GO:0051764",
  "gene_symbol": "GAS2L1",
  "gene_name": "GAS2-like protein 1",
  "term_label": "actin crosslink formation"
}